{
  "term_id": "GO:0006357",
  "gene_name": "Forkhead box protein P2",
  "term_label": "regulation of transcription by RNA polymerase II",
  "gene": "UniProtKB:O15409",
  "gene_symbol": "FOXP2"
}